{
  "term_label": "sodium ion transmembrane transport",
  "gene_symbol": "SCN2A",
  "gene": "UniProtKB:Q99250",
  "gene_name": "Sodium channel protein type 2 subunit alpha",
  "term_id": "GO:0035725"
}